cortical actin cytoskeleton organization [GO:0030866] (biological process) Also known as: actin cortex stabilization, cortical actin cytoskeleton organisation, cortical actin cytoskeleton stabilization, cortical actin cytoskeleton organization and biogenesis, cortical resistance Sources: GOC:dph, GOC:jl, GOC:mah, GOC:pf Definition: A process that is carried out at the cellular level which results in the assembly, arrangement of constituent parts, or disassembly of actin-based cytoskeletal structures in the cell cortex, i.e. just beneath the plasma membrane. Subtypes: actin cortical patch assembly [GO:0000147], GO:0044837, assembly of apicomedial cortex actomyosin [GO:0106036], terminal web assembly [GO:1902896] Relationships: is a type of actin cytoskeleton organization [GO:0030036]; is a type of GO:0030865